{
  "gene": "UniProtKB:Q5T4B2",
  "term_label": "Unknown cellular component",
  "term_id": "UNKNOWN:0003",
  "gene_symbol": "CERCAM",
  "gene_name": "Inactive glycosyltransferase 25 family member 3"
}